positive regulation of Frizzled Nuclear Import pathway [GO:0140711] (BP) References: PMID:22510459, PMID:22579286 Also known as: positive regulation of FNI, positive regulation of Frizzled Nuclear Import Wnt Pathway Definition: Any process that activates or increases the frequency, rate or extent of a Frizzled Nuclear Import pathway. Relationships: is a type of regulation of Frizzled Nuclear Import pathway [GO:0140710]; is a type of positive regulation of non-canonical Wnt signaling pathway [GO:2000052]; positively regulates Frizzled Nuclear Import pathway [GO:0140709]